{
  "gene_symbol": "SPO11",
  "gene": "UniProtKB:Q9Y5K1",
  "term_label": "meiotic DNA double-strand break processing",
  "term_id": "GO:0000706",
  "gene_name": "Meiotic recombination protein SPO11"
}